{
  "gene_name": "Cytochrome c oxidase subunit 7A-related protein, mitochondrial",
  "gene_symbol": "COX7A2L",
  "term_label": "protein-macromolecule adaptor activity",
  "term_id": "GO:0030674",
  "gene": "UniProtKB:O14548"
}